type 3 proteinase activated receptor binding [GO:0031874] (molecular function) Relationships: is a type of proteinase activated receptor binding [GO:0031871] Also known as: type 3 proteinase activated receptor ligand Sources: GOC:mah, GOC:nln Definition: Binding to a type 3 proteinase activated receptor.